{
  "gene": "UniProtKB:Q04828",
  "gene_symbol": "AKR1C1",
  "term_id": "GO:0044597",
  "gene_name": "Aldo-keto reductase family 1 member C1",
  "term_label": "daunorubicin metabolic process"
}